{
  "term_label": "extracellular matrix structural constituent conferring tensile strength",
  "gene_name": "Collagen alpha-2(IV) chain",
  "gene_symbol": "COL4A2",
  "term_id": "GO:0030020",
  "gene": "UniProtKB:P08572"
}